{
  "term_id": "GO:0043122",
  "gene": "UniProtKB:Q13077",
  "term_label": "regulation of canonical NF-kappaB signal transduction",
  "gene_symbol": "TRAF1",
  "gene_name": "TNF receptor-associated factor 1"
}